G/T mismatch-specific thymine-DNA glycosylase activity [GO:0141016] (molecular function) Relationships: is a type of pyrimidine-specific mismatch base pair DNA N-glycosylase activity [GO:0008263] Definition: Hydrolyzes mismatched double-stranded DNA and polynucleotides, releasing free thymine and leaving an apyrimidinic (AP) site. References: PMID:12711670 Sources: EC:3.2.2.29